{
  "term_label": "protein kinase binding",
  "term_id": "GO:0019901",
  "gene_name": "Putative speedy protein-like protein 3",
  "gene_symbol": "A6NJR5",
  "gene": "UniProtKB:A6NJR5"
}